{
  "term_label": "carotenoid dioxygenase activity",
  "gene": "UniProtKB:Q9BYV7",
  "gene_symbol": "BCO2",
  "term_id": "GO:0010436",
  "gene_name": "Carotenoid-cleaving dioxygenase, mitochondrial"
}